preprophase band [GO:0009574] (cellular component) Definition: A dense band of microtubules, 1-3 pm wide, that appears just beneath the cell membrane before the start of cell division in the cells of higher plants. It precedes the onset of prophase and then disappears as mitosis begins, yet it somehow determines the plane of orientation of the new cell plate forming in late telophase and marks the zone of the parental cell wall where fusion with the growing cell plate ultimately occurs. Sources: ISBN:0198506732 Relationships: is a type of cellular anatomical structure [GO:0110165]; is part of cytoplasm [GO:0005737]; is part of microtubule cytoskeleton [GO:0015630]